{
  "term_label": "DNA damage response",
  "gene": "UniProtKB:A0AVT1",
  "term_id": "GO:0006974",
  "gene_symbol": "UBA6",
  "gene_name": "Ubiquitin-like modifier-activating enzyme 6"
}